{
  "gene": "UniProtKB:Q9UNX3",
  "term_id": "GO:0002181",
  "gene_symbol": "RPL26L1",
  "gene_name": "Ribosomal protein uL24-like",
  "term_label": "cytoplasmic translation"
}